{
  "gene": "UniProtKB:Q8NGJ8",
  "term_label": "Unknown biological process",
  "gene_symbol": "OR51S1",
  "term_id": "UNKNOWN:0002",
  "gene_name": "Olfactory receptor 51S1"
}